{
  "term_id": "GO:0005634",
  "gene": "UniProtKB:A6NDR6",
  "gene_name": "Putative homeobox protein Meis3-like 1",
  "gene_symbol": "MEIS3P1",
  "term_label": "nucleus"
}